{
  "gene_name": "Fibroblast growth factor 4",
  "term_id": "GO:0008284",
  "term_label": "positive regulation of cell population proliferation",
  "gene": "UniProtKB:P08620",
  "gene_symbol": "FGF4"
}